{
  "term_id": "GO:0005886",
  "gene_symbol": "SLC9C1",
  "term_label": "plasma membrane",
  "gene_name": "Sodium_hydrogen exchanger 10",
  "gene": "UniProtKB:Q4G0N8"
}